{
  "gene_symbol": "SYNGR3",
  "gene_name": "Synaptogyrin-3",
  "term_id": "UNKNOWN:0002",
  "term_label": "Unknown biological process",
  "gene": "UniProtKB:O43761"
}